{
  "term_id": "GO:0022857",
  "gene_name": "Anion exchange protein 2",
  "gene_symbol": "SLC4A2",
  "gene": "UniProtKB:P04920",
  "term_label": "transmembrane transporter activity"
}